cytochrome complex assembly [GO:0017004] (biological process) Also known as: cytochrome biogenesis Sources: GOC:jl, GOC:mah Subtypes: respiratory chain complex IV assembly [GO:0008535], cytochrome b6f complex assembly [GO:0010190], respiratory chain complex III assembly [GO:0017062], cytochrome c-heme linkage [GO:0018063], protein-heme P460 linkage [GO:0018174], peroxidase-heme linkage [GO:0018186] Definition: The aggregation, arrangement and bonding together of a cytochrome complex. A cytochrome complex is a protein complex in which at least one of the proteins is a cytochrome, i.e. a heme-containing protein involved in catalysis of redox reactions. Relationships: is a type of protein-containing complex assembly [GO:0065003]